{
  "term_label": "positive regulation of synapse assembly",
  "term_id": "GO:0051965",
  "gene_symbol": "LRRTM4",
  "gene_name": "Leucine-rich repeat transmembrane neuronal protein 4",
  "gene": "UniProtKB:Q86VH4"
}